{
  "gene_symbol": "RBM24",
  "term_id": "GO:0005634",
  "gene": "UniProtKB:Q9BX46",
  "gene_name": "RNA-binding protein 24",
  "term_label": "nucleus"
}